{
  "gene": "UniProtKB:Q9H201",
  "term_label": "clathrin binding",
  "term_id": "GO:0030276",
  "gene_symbol": "EPN3",
  "gene_name": "Epsin-3"
}